{
  "gene_name": "Eukaryotic translation initiation factor 5A-2",
  "gene": "UniProtKB:Q9GZV4",
  "gene_symbol": "EIF5A2",
  "term_id": "GO:0006414",
  "term_label": "translational elongation"
}